{
  "gene_name": "E3 ubiquitin-protein ligase MARCHF9",
  "term_id": "GO:0004842",
  "term_label": "ubiquitin-protein transferase activity",
  "gene_symbol": "MARCHF9",
  "gene": "UniProtKB:Q86YJ5"
}